EFF-1 complex [GO:1990392] (cellular component) Definition: A trimeric cell-cell fusion complex that serves as a scaffold for zippering up the extracellular domains, bringing the transmembrane segments into close proximity such that they can continue zippering within the two membranes into one. Two prefusion monomers cluster at the surface of adjacent cells. Parallel EFF-1 interactions occur across cells and a third monomer, which can come from either cell, adds on to make an intermediate, extended trimer. References: PMID:24725407 Sources: GOC:bhm Relationships: is a type of plasma membrane protein complex [GO:0098797] Note: An example of this is eff-1 in C. elegans (G5ECA1) in PMID:24725407 (inferred from direct assay).